{
  "gene_name": "Cyclic GMP-AMP synthase",
  "gene_symbol": "CGAS",
  "term_id": "GO:0038001",
  "gene": "UniProtKB:Q8N884",
  "term_label": "paracrine signaling"
}